Kv4.2-KChIP1 channel complex [GO:0071192] (cellular component) Definition: A voltage-gated potassium channel complex that contains the Kv channel interacting protein KChIP1 associated with the channel via interaction with the Kv alpha subunit 4.2. References: PMID:15356203 Relationships: is a type of voltage-gated potassium channel complex [GO:0008076]